{
  "gene": "UniProtKB:Q9NRD8",
  "gene_name": "Dual oxidase 2",
  "term_id": "GO:0016174",
  "gene_symbol": "DUOX2",
  "term_label": "NAD(P)H oxidase H2O2-forming activity"
}